{
  "gene_name": "Thyroid hormone-inducible hepatic protein",
  "term_id": "GO:0046890",
  "term_label": "regulation of lipid biosynthetic process",
  "gene": "UniProtKB:Q92748",
  "gene_symbol": "THRSP"
}